response to raffinose [GO:1901545] (biological process) Relationships: is a type of response to carbohydrate [GO:0009743] Sources: GOC:TermGenie Subtypes: cellular response to raffinose [GO:0097403] Definition: Any process that results in a change in state or activity of a cell or an organism (in terms of movement, secretion, enzyme production, gene expression, etc.) as a result of a raffinose stimulus.